{
  "term_id": "GO:0007224",
  "term_label": "smoothened signaling pathway",
  "gene": "UniProtKB:O60291",
  "gene_symbol": "MGRN1",
  "gene_name": "E3 ubiquitin-protein ligase MGRN1"
}